{
  "term_id": "GO:0005516",
  "term_label": "calmodulin binding",
  "gene_name": "Calcium_calmodulin-dependent protein kinase type 1",
  "gene": "UniProtKB:Q14012",
  "gene_symbol": "CAMK1"
}